{
  "gene_symbol": "ATP6V1E1",
  "term_label": "Unknown cellular component",
  "gene": "UniProtKB:P36543",
  "gene_name": "V-type proton ATPase subunit E 1",
  "term_id": "UNKNOWN:0003"
}